{
  "gene_name": "Protocadherin beta-1",
  "term_label": "plasma membrane",
  "gene": "UniProtKB:Q9Y5F3",
  "term_id": "GO:0005886",
  "gene_symbol": "PCDHB1"
}